thiosulfate transmembrane transporter activity [GO:0015117] (MF) Definition: Enables the transfer of thiosulfate ions, HS2O3(1-), from one side of a membrane to the other. Sources: GOC:ai Also known as: thiosulphate transporter activity, thiosulfate permease activity Relationships: is a type of sulfur compound transmembrane transporter activity [GO:1901682]; is part of thiosulfate transport [GO:0015709] Subtypes: GO:0102025